{
  "gene_symbol": "BARX1",
  "gene_name": "Homeobox protein BarH-like 1",
  "term_label": "nucleus",
  "gene": "UniProtKB:Q9HBU1",
  "term_id": "GO:0005634"
}